{
  "term_id": "GO:0000122",
  "gene_name": "Zinc finger protein 572",
  "gene": "UniProtKB:Q7Z3I7",
  "term_label": "negative regulation of transcription by RNA polymerase II",
  "gene_symbol": "ZNF572"
}